protein phosphatase 5 binding [GO:1990634] (molecular function) References: PMID:8943293 Definition: Binding to protein phosphatase 5. Also known as: protein phosphatase T binding Relationships: is a type of GO:0019903